ajugose biosynthetic process [GO:0033536] (BP) Sources: GOC:mah Subtypes: ajugose biosynthetic process using galactinol:raffinose galactosyltransferase [GO:0033537], ajugose biosynthetic process using galactan:galactan galactosyltransferase [GO:0033538] Also known as: ajugose anabolism, ajugose biosynthesis, ajugose formation, ajugose synthesis Relationships: is_a GO:0010325 Definition: The chemical reactions and pathways resulting in the formation of ajugose, the hexasaccharide beta-D-fructofuranosyl alpha-D-galactopyranosyl-(1->6)-alpha-D-galactopyranosyl-(1->6)-alpha-D-galactopyranosyl-(1->6)-alpha-D-galactopyranosyl-(1->6)-alpha-D-glucopyranoside.